{
  "term_label": "G protein-coupled serotonin receptor activity",
  "gene_symbol": "HTR1B",
  "gene": "UniProtKB:P28222",
  "term_id": "GO:0004993",
  "gene_name": "5-hydroxytryptamine receptor 1B"
}